mesoderm migration involved in gastrulation [GO:0007509] (biological process) Definition: The migration of mesodermal cells during gastrulation to help establish the multilayered body plan of the organism. Relationships: is a type of mesodermal cell migration [GO:0008078]; is a type of cell migration involved in gastrulation [GO:0042074]; is a type of tissue migration [GO:0090130]; is part of mesoderm formation [GO:0001707] Sources: GOC:isa_complete, GOC:sat